negative regulation of maintenance of meiotic sister chromatid cohesion, centromeric [GO:2000710] (biological process) Sources: GOC:mah Definition: Any process that stops, prevents or reduces the frequency, rate or extent of maintenance of meiotic sister chromatid cohesion in the centromeric region. Also known as: negative regulation of maintenance of centromeric meiotic sister chromatin cohesion, negative regulation of maintenance of meiotic sister chromatin cohesion at centromere, negative regulation of maintenance of sister chromatin cohesion at centromere at meiosis I Relationships: is a type of negative regulation of maintenance of meiotic sister chromatid cohesion [GO:0034095]; is_a regulation of maintenance of meiotic sister chromatid cohesion, centromeric [GO:2000709]; negatively regulates maintenance of meiotic sister chromatid cohesion, centromeric [GO:0035875]